{
  "gene": "UniProtKB:P01906",
  "term_label": "MHC class II protein complex binding",
  "term_id": "GO:0023026",
  "gene_name": "HLA class II histocompatibility antigen, DQ alpha 2 chain",
  "gene_symbol": "HLA-DQA2"
}